{
  "gene_name": "N-terminal Xaa-Pro-Lys N-methyltransferase 1",
  "gene_symbol": "NTMT1",
  "term_id": "GO:0005737",
  "term_label": "cytoplasm",
  "gene": "UniProtKB:Q9BV86"
}